{
  "term_id": "GO:0005815",
  "gene": "UniProtKB:Q5T5M9",
  "gene_symbol": "CCNJ",
  "gene_name": "Cyclin-J",
  "term_label": "microtubule organizing center"
}